positive regulation of intestinal absorption [GO:1904480] (biological process) Also known as: up regulation of intestinal absorption, up-regulation of intestinal absorption, upregulation of intestinal absorption, activation of intestinal absorption Relationships: is a type of positive regulation of digestive system process [GO:0060456]; is a type of regulation of intestinal absorption [GO:1904478]; positively regulates intestinal absorption [GO:0050892] Subtypes: positive regulation of intestinal lipid absorption [GO:1904731] References: PMID:12469120 Sources: GOC:BHF, GOC:TermGenie, GOC:rl, GO_REF:0000058 Definition: Any process that activates or increases the frequency, rate or extent of intestinal absorption.